{
  "gene_symbol": "CHST6",
  "term_label": "N-acetylglucosamine 6-O-sulfotransferase activity",
  "gene_name": "Carbohydrate sulfotransferase 6",
  "gene": "UniProtKB:Q9GZX3",
  "term_id": "GO:0001517"
}